{
  "gene_symbol": "ANKS1B",
  "term_label": "ephrin receptor signaling pathway",
  "gene": "UniProtKB:Q7Z6G8",
  "term_id": "GO:0048013",
  "gene_name": "Ankyrin repeat and sterile alpha motif domain-containing protein 1B"
}